{
  "gene": "UniProtKB:Q15834",
  "term_label": "nucleus",
  "term_id": "GO:0005634",
  "gene_symbol": "CCDC85B",
  "gene_name": "Coiled-coil domain-containing protein 85B"
}